tertiary branching involved in mammary gland duct morphogenesis [GO:0060748] (biological process) Relationships: is a type of developmental process involved in reproduction [GO:0003006]; is part of GO:0060745 Definition: The branching process in which the mammary gland ducts form tertiary branches off of the secondary branches as part of diestrus and pregnancy. References: PMID:18614704 Sources: GOC:dph